{
  "gene_name": "Olfactory receptor 4Q2",
  "term_label": "Unknown biological process",
  "gene_symbol": "OR4Q2",
  "gene": "UniProtKB:P0C623",
  "term_id": "UNKNOWN:0002"
}